positive regulation of type I hypersensitivity [GO:0001812] (biological process) Definition: Any process that activates or increases the frequency, rate or extent of type I hypersensitivity, a type of inflammatory response. Sources: GOC:add, ISBN:0781735149 Also known as: up regulation of type I hypersensitivity, up-regulation of type I hypersensitivity, upregulation of type I hypersensitivity, activation of type I hypersensitivity, stimulation of type I hypersensitivity Relationships: is a type of regulation of type I hypersensitivity [GO:0001810]; is a type of positive regulation of hypersensitivity [GO:0002885]; is a type of positive regulation of immunoglobulin mediated immune response [GO:0002891]; positively regulates type I hypersensitivity [GO:0016068]